{
  "term_label": "Unknown molecular function",
  "gene": "UniProtKB:Q9NYZ1",
  "gene_symbol": "TVP23B",
  "term_id": "UNKNOWN:0001",
  "gene_name": "Golgi apparatus membrane protein TVP23 homolog B"
}